{
  "term_label": "Unknown biological process",
  "gene": "UniProtKB:P41732",
  "gene_name": "Tetraspanin-7",
  "gene_symbol": "TSPAN7",
  "term_id": "UNKNOWN:0002"
}